coenzyme B biosynthetic process [GO:0019298] (biological process) Definition: The chemical reactions and pathways resulting in the formation of coenzyme B (7-mercaptoheptanoylthreonine phosphate), a coenzyme involved in the utilization of methane by methanogenic prokaryotes. References: PMID:10940051 Also known as: coenzyme B anabolism, coenzyme B biosynthesis, coenzyme B formation, coenzyme B synthesis Relationships: is a type of phosphorus metabolic process [GO:0006793]; is a type of GO:0042398; is a type of monocarboxylic acid biosynthetic process [GO:0072330]